{
  "gene_name": "Transforming growth factor-beta receptor-associated protein 1",
  "gene": "UniProtKB:Q8WUH2",
  "gene_symbol": "TGFBRAP1",
  "term_id": "UNKNOWN:0001",
  "term_label": "Unknown molecular function"
}